{
  "gene_name": "Nuclear receptor subfamily 2 group C member 2",
  "gene": "UniProtKB:P49116",
  "gene_symbol": "NR2C2",
  "term_label": "nuclear receptor activity",
  "term_id": "GO:0004879"
}